maintenance of protein location in nucleus [GO:0051457] (biological process) Definition: Any process in which a protein is maintained in the nucleus and prevented from moving elsewhere. These include sequestration within the nucleus, protein stabilization to prevent transport elsewhere and the active retrieval of proteins that escape the nucleus. Also known as: maintenance of nuclear protein localization, maintenance of protein location in cell nucleus, nuclear protein retention, nuclear protein sequestering, nuclear protein sequestration, protein retention in nucleus, protein sequestration in nucleus, protein storage in nucleus, protein-nuclear retention, sequestration of protein in nucleus, storage of protein in nucleus, maintenance of protein localization in nucleus Relationships: is a type of maintenance of protein localization in organelle [GO:0072595]; is part of protein localization to nucleus [GO:0034504]; occurs in GO:0005634 Sources: GOC:ai Subtypes: negative regulation of protein export from nucleus [GO:0046826], GO:0090292